galacturonate transmembrane transport [GO:0015737] (biological process) Definition: The process in which galacturonate is transported across a lipid bilayer, from one side of a membrane to the other. Sources: GOC:krc Also known as: galacturonate transport Relationships: is a type of hexuronate transmembrane transport [GO:0015736]